{
  "gene_name": "Enhancer of filamentation 1",
  "gene_symbol": "NEDD9",
  "term_label": "cell migration",
  "term_id": "GO:0016477",
  "gene": "UniProtKB:Q14511"
}